positive regulation of calcium ion import across plasma membrane [GO:1905665] (biological process) Note: An example of this is PPP3CA in human (Q08209) in 17640527 (inferred from direct assay). References: PMID:17640527 Sources: GOC:TermGenie, GOC:bhm, GO_REF:0000058 Definition: Any process that activates or increases the frequency, rate or extent of calcium ion import across plasma membrane. Also known as: up regulation of calcium ion import across plasma membrane, up-regulation of calcium ion import across plasma membrane, upregulation of calcium ion import across plasma membrane, activation of calcium ion import across plasma membrane Relationships: is a type of GO:0090280; is a type of positive regulation of calcium ion transmembrane transport [GO:1904427]; is a type of regulation of calcium ion import across plasma membrane [GO:1905664]; RO_0002213 calcium ion import across plasma membrane [GO:0098703]